{
  "gene_symbol": "FGF6",
  "gene": "UniProtKB:P10767",
  "term_id": "GO:0008543",
  "term_label": "fibroblast growth factor receptor signaling pathway",
  "gene_name": "Fibroblast growth factor 6"
}